NADH binding [GO:0070404] (MF) Sources: GOC:mah Definition: Binding to the reduced form, NADH, of nicotinamide adenine dinucleotide, a coenzyme involved in many redox and biosynthetic reactions. Relationships: is a type of anion binding [GO:0043168]; is a type of NAD binding [GO:0051287] Also known as: NAD (reduced) binding, reduced NAD binding, reduced nicotinamide adenine dinucleotide binding